proline metabolic process [GO:0006560] (biological process) Subtypes: L-proline catabolic process [GO:0006562], L-ornithine catabolic process via proline [GO:0019466], L-arginine catabolic process to L-proline [GO:0019493], GO:0055129 Definition: The chemical reactions and pathways involving proline (pyrrolidine-2-carboxylic acid), a chiral, cyclic, nonessential alpha-amino acid found in peptide linkage in proteins. Sources: GOC:jl, ISBN:0198506732 Relationships: is a type of glutamine family amino acid metabolic process [GO:0009064] Also known as: proline metabolism Regulation: regulated by regulation of L-proline metabolic process [GO:2000214]